{
  "term_id": "GO:0016251",
  "term_label": "RNA polymerase II general transcription initiation factor activity",
  "gene_symbol": "TAF7L",
  "gene": "UniProtKB:Q5H9L4",
  "gene_name": "Transcription initiation factor TFIID subunit 7-like"
}